cis assembly of pre-catalytic spliceosome [GO:0000354] (BP) Definition: Assembly of a spliceosomal complex containing the intact pre-mRNA and all of the spliceosomal snRNPs. This occurs when the tri-snRNP associates with the pre-mRNA and associated snRNPs in an ATP-dependent manner. Also known as: cis assembly of U12-type pre-catalytic spliceosome, cis assembly of U2-type pre-catalytic spliceosome, formation of spliceosomal A2-1 complex, formation of spliceosomal B1 complex, spliceosomal A2-1 complex biosynthesis, spliceosomal A2-1 complex formation, spliceosomal B1 complex biosynthesis, spliceosomal B1 complex formation Sources: GOC:krc, GOC:mtg_mpo, ISBN:0879695897 Note: Note that this step represents formation of the A2-1 complex (yeast) or the B1 complex (mammals). Relationships: is_a protein-RNA complex assembly [GO:0022618]; BFO_0000050 GO:0000245; is part of mRNA cis splicing, via spliceosome [GO:0045292]